{
  "gene": "UniProtKB:Q9Y6X9",
  "gene_symbol": "MORC2",
  "term_id": "UNKNOWN:0002",
  "term_label": "Unknown biological process",
  "gene_name": "ATPase MORC2"
}